{
  "gene": "UniProtKB:O95834",
  "term_label": "microtubule binding",
  "gene_symbol": "EML2",
  "gene_name": "Echinoderm microtubule-associated protein-like 2",
  "term_id": "GO:0008017"
}